{
  "term_label": "cytosol",
  "term_id": "GO:0005829",
  "gene_name": "Serine_threonine-protein kinase Nek6",
  "gene_symbol": "NEK6",
  "gene": "UniProtKB:Q9HC98"
}